{
  "gene_name": "Synapse differentiation-inducing gene protein 1",
  "gene": "UniProtKB:Q9H7V2",
  "gene_symbol": "SYNDIG1",
  "term_label": "postsynaptic density membrane",
  "term_id": "GO:0098839"
}